diaminobutyrate-2-oxoglutarate transaminase activity [GO:0045303] (molecular function) Sources: EC:2.6.1.76, RHEA:11160 Relationships: is a type of transaminase activity [GO:0008483] Also known as: 2,4-diaminobutyrate 4-aminotransferase activity, DAB aminotransferase activity, DABA aminotransferase activity, EctB, L-2,4-diaminobutanoate:2-oxoglutarate 4-aminotransferase activity, L-2,4-diaminobutyrate:2-ketoglutarate 4-aminotransferase activity, L-2,4-diaminobutyrate:2-oxoglutarate 4-aminotransferase activity, diaminibutyric acid aminotransferase activity, diaminobutyrate transaminase activity, diaminobutyrate--2-oxoglutarate aminotransferase activity Definition: Catalysis of the reaction: 2-oxoglutarate + L-2,4-diaminobutyrate = L-aspartate 4-semialdehyde + L-glutamate.